otic vesicle formation [GO:0030916] (biological process) Also known as: otocyst biosynthesis, otocyst formation Relationships: is a type of epithelial tube formation [GO:0072175]; is part of otic vesicle morphogenesis [GO:0071600] Definition: The process resulting in the transition of the otic placode into the otic vesicle, a transient embryonic structure formed during development of the vertebrate inner ear. Sources: GOC:dgh